{
  "gene_name": "Keratin-associated protein 5-7",
  "term_label": "Unknown biological process",
  "gene": "UniProtKB:Q6L8G8",
  "gene_symbol": "KRTAP5-7",
  "term_id": "UNKNOWN:0002"
}